{
  "gene": "UniProtKB:P41159",
  "gene_symbol": "LEP",
  "gene_name": "Leptin",
  "term_label": "extracellular space",
  "term_id": "GO:0005615"
}